{
  "term_id": "GO:0000145",
  "gene_symbol": "EXOC7",
  "term_label": "exocyst",
  "gene": "UniProtKB:Q9UPT5",
  "gene_name": "Exocyst complex component 7"
}